{
  "gene_name": "Ankyrin repeat domain-containing protein 9",
  "term_label": "Unknown biological process",
  "gene": "UniProtKB:Q96BM1",
  "term_id": "UNKNOWN:0002",
  "gene_symbol": "ANKRD9"
}